{
  "term_id": "GO:0061578",
  "gene_name": "AMSH-like protease",
  "gene_symbol": "STAMBPL1",
  "gene": "UniProtKB:Q96FJ0",
  "term_label": "K63-linked deubiquitinase activity"
}